{
  "gene_symbol": "MARVELD2",
  "gene": "UniProtKB:Q8N4S9",
  "term_label": "cytoplasmic vesicle",
  "term_id": "GO:0031410",
  "gene_name": "MARVEL domain-containing protein 2"
}